fibroblast growth factor receptor signaling pathway involved in hemopoiesis [GO:0035603] (biological process) Sources: GOC:yaf Definition: The series of molecular signals generated as a consequence of a fibroblast growth factor receptor binding to one of its physiological ligands, which contributes to hemopoiesis. Relationships: is a type of fibroblast growth factor receptor signaling pathway [GO:0008543]; is part of hemopoiesis [GO:0030097] Also known as: FGF receptor signaling pathway involved in hematopoiesis, FGFR signaling pathway involved in hematopoiesis, fibroblast growth factor receptor signaling pathway involved in hematopoiesis, fibroblast growth factor receptor signalling pathway involved in hemopoiesis